embryonic ectodermal digestive tract development [GO:0048611] (biological process) Definition: The process, occurring during the embryonic phase, whose specific outcome is the progression of the ectodermal gut over time, from its formation to the mature structure. Sources: GOC:jid, GOC:rc Relationships: is a type of embryonic digestive tract development [GO:0048566]; is part of GO:0007439 Also known as: embryonic ectodermal gut development